{
  "gene_symbol": "PARVG",
  "term_label": "cell projection assembly",
  "gene": "UniProtKB:Q9HBI0",
  "term_id": "GO:0030031",
  "gene_name": "Gamma-parvin"
}